{
  "gene": "UniProtKB:P0DTU3",
  "term_label": "Unknown molecular function",
  "gene_symbol": "TRA",
  "gene_name": "T cell receptor alpha chain MC.7.G5",
  "term_id": "UNKNOWN:0001"
}